{
  "term_id": "UNKNOWN:0001",
  "gene_name": "Peptidyl-prolyl cis-trans isomerase NIMA-interacting 4",
  "gene": "UniProtKB:Q9Y237",
  "term_label": "Unknown molecular function",
  "gene_symbol": "PIN4"
}